{
  "term_label": "Unknown biological process",
  "term_id": "UNKNOWN:0002",
  "gene_name": "Membrane progestin receptor epsilon",
  "gene": "UniProtKB:Q6ZVX9",
  "gene_symbol": "PAQR9"
}